{
  "gene_name": "Fanconi-associated nuclease 1",
  "gene_symbol": "FAN1",
  "term_id": "GO:0005634",
  "term_label": "nucleus",
  "gene": "UniProtKB:Q9Y2M0"
}